{
  "gene": "UniProtKB:Q9UBQ6",
  "term_label": "Unknown biological process",
  "gene_name": "Exostosin-like 2",
  "gene_symbol": "EXTL2",
  "term_id": "UNKNOWN:0002"
}